{
  "term_label": "cell surface receptor signaling pathway",
  "gene": "UniProtKB:A0A0B4J2E0",
  "term_id": "GO:0007166",
  "gene_name": "T cell receptor beta variable 12-4",
  "gene_symbol": "TRBV12-4"
}